cytosolic translation preinitiation complex [GO:0070993] (cellular component) Definition: A ribonucleoprotein complex that contains the small ribosomal subunit, a translation initiation ternary complex (i.e. an initiator tRNA, GTP, and an IF2 or eIF2 complex), and an mRNA. Relationships: is a type of ribonucleoprotein complex [GO:1990904]; is part of GO:0005737 Sources: GOC:hjd, GOC:mah Subtypes: GO:0016282, eukaryotic 48S preinitiation complex [GO:0033290]